axon [GO:0030424] (cellular component) Definition: The long process of a neuron that conducts nerve impulses, usually away from the cell body to the terminals and varicosities, which are sites of storage and release of neurotransmitter. Subtypes: GO:0042757, C-fiber [GO:0044299], GO:0044300, climbing fiber [GO:0044301], GO:0097457, parallel fiber [GO:1990032] Relationships: is a type of neuron projection [GO:0043005] Sources: GOC:nln, ISBN:0198506732